{
  "gene_name": "Fez family zinc finger protein 1",
  "gene": "UniProtKB:A0PJY2",
  "term_id": "GO:0006357",
  "term_label": "regulation of transcription by RNA polymerase II",
  "gene_symbol": "FEZF1"
}